{
  "term_label": "nucleus",
  "term_id": "GO:0005634",
  "gene_name": "Actin-related protein T1",
  "gene_symbol": "ACTRT1",
  "gene": "UniProtKB:Q8TDG2"
}